{
  "gene_symbol": "SIGLEC9",
  "term_label": "sialic acid binding",
  "gene": "UniProtKB:Q9Y336",
  "term_id": "GO:0033691",
  "gene_name": "Sialic acid-binding Ig-like lectin 9"
}